{
  "term_id": "GO:0005737",
  "gene_name": "Serine_threonine-protein kinase 3",
  "term_label": "cytoplasm",
  "gene_symbol": "STK3",
  "gene": "UniProtKB:Q13188"
}